{
  "gene_name": "Exonuclease V",
  "term_label": "single-stranded DNA 5'-3' DNA exonuclease activity",
  "gene": "UniProtKB:Q9H790",
  "term_id": "GO:0045145",
  "gene_symbol": "EXO5"
}